{
  "term_id": "UNKNOWN:0001",
  "gene_name": "Signal peptide, CUB and EGF-like domain-containing protein 2",
  "gene": "UniProtKB:Q9NQ36",
  "term_label": "Unknown molecular function",
  "gene_symbol": "SCUBE2"
}